regulation of natural killer cell degranulation [GO:0043321] (biological process) Also known as: regulation of NK cell degranulation, regulation of NK cell granule exocytosis, regulation of natural killer cell granule exocytosis Subtypes: GO:0043322, GO:0043323 Sources: ISBN:0781735149 Definition: Any process that modulates the frequency, rate, or extent of natural killer cell degranulation. Relationships: is a type of GO:0042269; is a type of regulation of leukocyte degranulation [GO:0043300]; regulates natural killer cell degranulation [GO:0043320]